regulation of establishment of protein localization to telomere [GO:0070203] (biological process) Sources: GOC:BHF, GOC:mah Relationships: is a type of regulation of establishment of protein localization to chromosome [GO:0070202]; regulates establishment of protein localization to telomere [GO:0070200] Also known as: regulation of establishment of protein localisation to telomere Subtypes: GO:1904850, positive regulation of establishment of protein localization to telomere [GO:1904851] Definition: Any process that modulates the frequency, rate or extent of the directed movement of a protein to a specific location in the telomeric region of a chromosome.